dCMP kinase activity [GO:0036431] (molecular function) Definition: Catalysis of the reaction: ATP + dCMP = ADP + dCDP. Sources: RHEA:25094 Also known as: ATP:dCMP phosphotransferase activity Relationships: is a type of deoxynucleoside phosphate kinase activity, ATP as phosphate donor [GO:0047507]